{
  "gene": "UniProtKB:O94919",
  "term_id": "UNKNOWN:0001",
  "term_label": "Unknown molecular function",
  "gene_name": "Endonuclease domain-containing 1 protein",
  "gene_symbol": "ENDOD1"
}